cornification [GO:0070268] (biological process) Regulation: regulated by regulation of cornification [GO:1905715]; negatively regulated by negative regulation of cornification [GO:1905716]; RO_0002213 by GO:1905717 Relationships: is a type of programmed cell death [GO:0012501]; is part of keratinization [GO:0031424]; has part cornified envelope assembly [GO:1903575] Definition: A type of programmed cell death that occurs in the epidermis, morphologically and biochemically distinct from apoptosis. It leads to the formation of corneocytes, i.e. dead keratinocytes containing an amalgam of specific proteins (e.g., keratin, loricrin, SPR and involucrin) and lipids (e.g., fatty acids and ceramides), which are necessary for the function of the cornified skin layer (mechanical resistance, elasticity, water repellence and structural stability). References: PMID:18846107 Sources: GOC:krc